{
  "gene": "UniProtKB:O75190",
  "gene_symbol": "DNAJB6",
  "term_id": "GO:0051082",
  "term_label": "unfolded protein binding",
  "gene_name": "DnaJ homolog subfamily B member 6"
}